{
  "gene_name": "Eukaryotic translation initiation factor 2-alpha kinase 1",
  "gene": "UniProtKB:Q9BQI3",
  "gene_symbol": "EIF2AK1",
  "term_label": "cytoplasm",
  "term_id": "GO:0005737"
}